{
  "gene_symbol": "OR2M3",
  "gene": "UniProtKB:Q8NG83",
  "term_label": "detection of chemical stimulus involved in sensory perception of smell",
  "gene_name": "Olfactory receptor 2M3",
  "term_id": "GO:0050911"
}